ventricular cardiac muscle cell membrane repolarization [GO:0099625] (biological process) Sources: GOC:BHF, GOC:mtg_cardiac_conduct_nov11 Definition: The process in which ions are transported across the plasma membrane of a ventricular cardiac muscle cell such that the membrane potential changes in the repolarizing direction, toward the steady state potential. For example, the repolarization during an action potential is from a positive membrane potential towards a negative resting potential. Regulation: regulated by regulation of ventricular cardiac muscle cell membrane repolarization [GO:0060307] Relationships: is a type of cardiac muscle cell membrane repolarization [GO:0099622] Subtypes: membrane repolarization during ventricular cardiac muscle cell action potential [GO:0098915]